{
  "term_label": "Unknown biological process",
  "gene_name": "Annexin A4",
  "gene_symbol": "ANXA4",
  "gene": "UniProtKB:P09525",
  "term_id": "UNKNOWN:0002"
}